{
  "gene": "UniProtKB:Q6UVY6",
  "gene_symbol": "MOXD1",
  "term_label": "dopamine beta-monooxygenase activity",
  "gene_name": "DBH-like monooxygenase protein 1",
  "term_id": "GO:0004500"
}